{
  "gene_symbol": "NRGN",
  "term_label": "Unknown cellular component",
  "term_id": "UNKNOWN:0003",
  "gene_name": "Neurogranin",
  "gene": "UniProtKB:Q92686"
}